{
  "gene_name": "Cdc42 effector protein 3",
  "gene_symbol": "CDC42EP3",
  "term_label": "small GTPase binding",
  "term_id": "GO:0031267",
  "gene": "UniProtKB:Q9UKI2"
}